positive regulation of satellite cell activation involved in skeletal muscle regeneration [GO:0014718] (biological process) Definition: Any process that activates, maintains or increases the frequency, rate or extent of activation of satellite cell involved in skeletal muscle regeneration. The activation of satellite cell is the process that initiates satellite cell division by causing it to move from quiescence to the G1 stage of the cell cycle. The cell swells and there are a number of other small changes. The cells then start to divide. Following cell division the cells will differentiate. Relationships: is a type of regulation of satellite cell activation involved in skeletal muscle regeneration [GO:0014717]; is a type of positive regulation of skeletal muscle tissue regeneration [GO:0043415]; is a type of positive regulation of cell activation [GO:0050867]; positively regulates satellite cell activation involved in skeletal muscle regeneration [GO:0014901] Sources: GOC:mtg_muscle